R3/R4 development [GO:0048057] (BP) Definition: The process whose specific outcome is the progression of the R3 and R4 pair of photoreceptors in the eye over time, from their formation to the mature structures. R3 and R4 are paired photoreceptors that contribute to the outer rhabdomeres. An example of this process is found in Drosophila melanogaster. Relationships: is a type of compound eye photoreceptor development [GO:0042051]; is part of GO:0048056 Sources: GOC:jid